{
  "gene_name": "Carboxypeptidase A5",
  "term_id": "GO:0005615",
  "term_label": "extracellular space",
  "gene_symbol": "CPA5",
  "gene": "UniProtKB:Q8WXQ8"
}